guanosine biosynthetic process [GO:0046114] (biological process) Relationships: is a type of guanosine metabolic process [GO:0008617]; is a type of guanosine-containing compound biosynthetic process [GO:1901070] Sources: GOC:go_curators Definition: The chemical reactions and pathways resulting in the formation of guanine, guanine riboside, a nucleoside with a wide species distribution. Subtypes: GO:0006179 Also known as: guanosine anabolism, guanosine biosynthesis, guanosine formation, guanosine synthesis